{
  "term_label": "antigen binding",
  "gene_name": "Immunoglobulin heavy variable 1-8",
  "term_id": "GO:0003823",
  "gene_symbol": "IGHV1-8",
  "gene": "UniProtKB:P0DP01"
}